mitochondrial complex I intermediate assembly complex [GO:0160295] (cellular component) Also known as: MCIA complex, mitochondrial CI assembly complex Relationships: is a type of inner mitochondrial membrane protein complex [GO:0098800] Definition: A protein complex involved in mitochondrial respiratory chain complex I (MCI) assembly. The mitochondrial complex I intermediate assembly (MCIA) complex is an inner mitochondrial membrane complex required for the aggregation, arrangement and bonding together of the subunits of the ND2-module of MCI. In humans, the MCIA complex is formed from NDUFAF1, ACAD9, ECSIT, TMEM126B, TMEM186 and COA1. References: PMID:32320651